{
  "gene_symbol": "CFAP97D1",
  "term_id": "UNKNOWN:0003",
  "gene_name": "Sperm axonemal maintenance protein CFAP97D1",
  "gene": "UniProtKB:B2RV13",
  "term_label": "Unknown cellular component"
}